{
  "gene_symbol": "GNAL",
  "gene": "UniProtKB:P38405",
  "term_label": "cytoplasm",
  "term_id": "GO:0005737",
  "gene_name": "Guanine nucleotide-binding protein G(olf) subunit alpha"
}